dendritic lamellar body [GO:1990503] (cellular component) Also known as: DLB References: PMID:7869120 Definition: A specialized secretory organelle found in neurons and associated with the formation of dendrodendritic gap junctions. Relationships: is a type of GO:0042599; is part of dendrite [GO:0030425]